{
  "term_label": "ATPase-coupled intramembrane lipid transporter activity",
  "gene_symbol": "ATP11A",
  "gene_name": "Phospholipid-transporting ATPase IH",
  "term_id": "GO:0140326",
  "gene": "UniProtKB:P98196"
}